{
  "gene_name": "Pregnancy zone protein",
  "gene": "UniProtKB:P20742",
  "gene_symbol": "PZP",
  "term_id": "GO:0004866",
  "term_label": "endopeptidase inhibitor activity"
}